thetin-homocysteine S-methyltransferase activity [GO:0047149] (molecular function) Also known as: dimethylsulfonioacetate:L-homocysteine S-methyltransferase activity, dimethylthetin-homocysteine methyltransferase activity, thetin-homocysteine methylpherase activity Sources: EC:2.1.1.3, RHEA:22788 Relationships: is a type of S-methyltransferase activity [GO:0008172] Definition: Catalysis of the reaction: L-homocysteine + dimethylsulfonioacetate = (methylthio)acetate + L-methionine + H+.